{
  "gene": "UniProtKB:Q9Y251",
  "gene_symbol": "HPSE",
  "term_label": "cell-matrix adhesion",
  "gene_name": "Heparanase",
  "term_id": "GO:0007160"
}